{
  "gene_name": "C-C chemokine receptor type 4",
  "gene_symbol": "CCR4",
  "term_label": "immune response",
  "gene": "UniProtKB:P51679",
  "term_id": "GO:0006955"
}